{
  "gene_name": "Neurotrimin",
  "term_id": "GO:0005886",
  "gene": "UniProtKB:Q9P121",
  "term_label": "plasma membrane",
  "gene_symbol": "NTM"
}